{
  "term_id": "GO:0090110",
  "term_label": "COPII-coated vesicle cargo loading",
  "gene_name": "Protein transport protein Sec31B",
  "gene_symbol": "SEC31B",
  "gene": "UniProtKB:Q9NQW1"
}